{
  "term_label": "extracellular matrix",
  "term_id": "GO:0031012",
  "gene": "UniProtKB:P35442",
  "gene_symbol": "THBS2",
  "gene_name": "Thrombospondin-2"
}